mesenchymal cell differentiation involved in kidney development [GO:0072161] (biological process) Definition: The process in which relatively unspecialized cells acquire specialized structural and/or functional features that characterize the mesenchymal cells of the kidney as it progresses from its formation to the mature state. Subtypes: mesonephric mesenchymal cell differentiation [GO:0061223], metanephric mesenchymal cell differentiation [GO:0072162] Sources: GOC:mtg_kidney_jan10 Relationships: is a type of cell differentiation involved in kidney development [GO:0061005]; is a type of mesenchymal cell differentiation involved in renal system development [GO:2001012]; is part of kidney mesenchyme development [GO:0072074]